{
  "gene": "UniProtKB:Q9H269",
  "gene_symbol": "VPS16",
  "gene_name": "Vacuolar protein sorting-associated protein 16 homolog",
  "term_id": "GO:0005768",
  "term_label": "endosome"
}